{
  "gene": "UniProtKB:Q8IUW3",
  "gene_symbol": "SPATA2L",
  "gene_name": "Spermatogenesis-associated protein 2-like protein",
  "term_id": "UNKNOWN:0001",
  "term_label": "Unknown molecular function"
}